{
  "gene": "UniProtKB:Q92569",
  "term_id": "GO:0046935",
  "gene_symbol": "PIK3R3",
  "term_label": "1-phosphatidylinositol-3-kinase regulator activity",
  "gene_name": "Phosphatidylinositol 3-kinase regulatory subunit gamma"
}